{
  "gene": "UniProtKB:Q9NVG8",
  "gene_symbol": "TBC1D13",
  "term_label": "cytoplasm",
  "term_id": "GO:0005737",
  "gene_name": "TBC1 domain family member 13"
}